{
  "term_label": "Unknown molecular function",
  "term_id": "UNKNOWN:0001",
  "gene": "UniProtKB:A0A1B0GTL2",
  "gene_name": "Uncharacterized protein C20orf204",
  "gene_symbol": "C20orf204"
}